azole transmembrane transport [GO:0045117] (biological process) Definition: The directed movement of azoles, heterocyclic compounds found in many biologically important substances, across a lipid bilayer, across a membrane. Sources: GOC:go_curators, ISBN:3527307206, Wikipedia:Azole Relationships: is a type of transmembrane transport [GO:0055085]; is a type of nitrogen compound transport [GO:0071705] Subtypes: thiamine transmembrane transport [GO:0071934], GO:0089709, sulfathiazole transmembrane transport [GO:1902599], 5-amino-1-ribofuranosylimidazole-4-carboxamide transmembrane transport [GO:1903088], GO:1905130 Also known as: azole transport